{
  "gene": "UniProtKB:O76095",
  "term_id": "GO:0000281",
  "gene_name": "Protein JTB",
  "gene_symbol": "JTB",
  "term_label": "mitotic cytokinesis"
}